{
  "gene": "UniProtKB:Q9BY07",
  "gene_symbol": "SLC4A5",
  "gene_name": "Electrogenic sodium bicarbonate cotransporter 4",
  "term_id": "GO:0051453",
  "term_label": "regulation of intracellular pH"
}